susceptibility to natural killer cell mediated cytotoxicity [GO:0042271] (biological process) Definition: The process of causing a cell to become susceptible to natural killer cell mediated cytotoxicity. Sources: GOC:add, ISBN:0781735149 Also known as: susceptibility to NK cell mediated cell death, susceptibility to NK cell mediated cell killing, susceptibility to NK cell mediated cytolysis, susceptibility to NK cell mediated cytotoxicity, susceptibility to natural killer cell mediated cell death, susceptibility to natural killer cell mediated cell killing, susceptibility to natural killer cell mediated cytolysis Note: Note that this term is intended for cell-surface molecules on a target cell which interact with activating receptors on a natural killer cell to promote natural killer cell mediated cytotoxicity. Relationships: is a type of positive regulation of natural killer cell mediated cytotoxicity [GO:0045954]